{
  "gene": "UniProtKB:O95178",
  "gene_symbol": "NDUFB2",
  "term_id": "GO:0045271",
  "term_label": "respiratory chain complex I",
  "gene_name": "NADH dehydrogenase [ubiquinone] 1 beta subcomplex subunit 2, mitochondrial"
}